{
  "gene": "UniProtKB:P34969",
  "gene_name": "5-hydroxytryptamine receptor 7",
  "term_id": "GO:0007268",
  "term_label": "chemical synaptic transmission",
  "gene_symbol": "HTR7"
}